Rho-activating G protein-coupled receptor signaling pathway [GO:0160221] (biological process) Relationships: is_a GO:0007186 Definition: A G protein-coupled receptor signaling pathway in which the signal is transmitted via the activation of Rho activity. Rho is a family of small (~21 kDa) signaling G proteins that include RhoA, Cdc42, and Rac1. References: PMID:10836144, PMID:33849392